{
  "term_id": "GO:0019864",
  "gene_symbol": "FCER1G",
  "gene": "UniProtKB:P30273",
  "gene_name": "High affinity immunoglobulin epsilon receptor subunit gamma",
  "term_label": "IgG binding"
}